entry of viral genome into host nucleus through nuclear pore complex via importin [GO:0075506] (biological process) Note: This mechanism is used by some RNA viruses (e.g. Orthomyxoviridae), some dsDNA viruses (e.g. Polyomaviridae) and some ssRNA viruses (e.g. Lentivirus). Also known as: entry of viral genome into host nucleus via cellular importin transport through the nuclear pore complex Relationships: is a type of GO:0075732 Definition: Viral penetration into the host nucleus where the viral genome passes through the nuclear pore complex (NPC) using the cellular importin transport machinery. References: PMID:22929056 Sources: VZ:989